{
  "gene_name": "ELKS_Rab6-interacting_CAST family member 1",
  "gene": "UniProtKB:Q8IUD2",
  "term_id": "GO:0098831",
  "gene_symbol": "ERC1",
  "term_label": "presynaptic active zone cytoplasmic component"
}